{
  "gene_name": "Large ribosomal subunit protein eL33",
  "term_label": "structural constituent of ribosome",
  "gene_symbol": "RPL35A",
  "term_id": "GO:0003735",
  "gene": "UniProtKB:P18077"
}